{
  "term_label": "integrin binding",
  "gene_symbol": "CCN1",
  "term_id": "GO:0005178",
  "gene_name": "CCN family member 1",
  "gene": "UniProtKB:O00622"
}